{
  "gene_name": "5-hydroxytryptamine receptor 1B",
  "gene": "UniProtKB:P28222",
  "gene_symbol": "HTR1B",
  "term_label": "adenylate cyclase-inhibiting serotonin receptor signaling pathway",
  "term_id": "GO:0007198"
}